N-carbamoyl-D-amino acid hydrolase activity [GO:0047417] (molecular function) Also known as: N-carbamoyl-D-amino acid amidohydrolase activity Definition: Catalysis of the reaction: H2O + N-carbamoyl-D-amino acid = CO2 + NH3 + D-amino acid. Sources: EC:3.5.1.77, MetaCyc:3.5.1.77-RXN Relationships: is a type of hydrolase activity, acting on carbon-nitrogen (but not peptide) bonds, in linear amides [GO:0016811]